cellular response to vitamin [GO:0071295] (biological process) Relationships: is a type of cellular response to nutrient [GO:0031670]; is a type of GO:0033273 Sources: GOC:mah Subtypes: GO:0071231, GO:0071296, cellular response to cobalamin [GO:0071297], cellular response to L-ascorbic acid [GO:0071298], cellular response to vitamin A [GO:0071299], GO:0071301, cellular response to vitamin B2 [GO:0071302], cellular response to vitamin B3 [GO:0071303], cellular response to vitamin B6 [GO:0071304], cellular response to vitamin D [GO:0071305], GO:0071306, cellular response to vitamin K [GO:0071307] Definition: Any process that results in a change in state or activity of a cell (in terms of movement, secretion, enzyme production, gene expression, etc.) as a result of a vitamin stimulus.